presynaptic active zone organization [GO:1990709] (biological process) Also known as: presynaptic active zone organisation Definition: A process that results in the assembly, arrangement of constituent parts, or disassembly of a presynaptic active zone. Relationships: is a type of cellular component organization [GO:0016043]; is part of GO:0050808 Subtypes: maintenance of presynaptic active zone structure [GO:0048790], GO:1904071, GO:1904072 References: PMID:16865347, PMID:17068967 Sources: GOC:pr